pigment granule aggregation in cell center [GO:0051877] (biological process) Sources: GOC:mh Definition: The directed movement of dispersed pigment granules towards the center of the cell. Relationships: is a type of establishment of pigment granule localization [GO:0051905]